{
  "gene_symbol": "NOD1",
  "gene_name": "Nucleotide-binding oligomerization domain-containing protein 1",
  "term_id": "GO:0042742",
  "gene": "UniProtKB:Q9Y239",
  "term_label": "defense response to bacterium"
}